{
  "term_id": "GO:0005886",
  "gene_name": "GEM-interacting protein",
  "term_label": "plasma membrane",
  "gene_symbol": "GMIP",
  "gene": "UniProtKB:Q9P107"
}